{
  "gene": "UniProtKB:Q9NZP5",
  "term_label": "olfactory receptor activity",
  "gene_symbol": "OR5AC2",
  "term_id": "GO:0004984",
  "gene_name": "Olfactory receptor 5AC2"
}